phosphate-containing compound metabolic process [GO:0006796] (biological process) Definition: The chemical reactions and pathways involving the phosphate group, the anion or salt of any phosphoric acid. Sources: GOC:ai Also known as: phosphate metabolism, phosphate metabolic process Relationships: is a type of phosphorus metabolic process [GO:0006793] Subtypes: fructose 6-phosphate metabolic process [GO:0006002], GO:0006003, phosphocreatine metabolic process [GO:0006603], GO:0006644, GO:0006753, GO:0016310, GO:0016311, glucose 1-phosphate metabolic process [GO:0019255], L-methionine biosynthetic process from L-homoserine via O-phospho-L-homoserine and cystathionine [GO:0019283], parathion catabolic process [GO:0019339], sucrose catabolic process via 3'-ketosucrose [GO:0019574], GO:0019664, glyceraldehyde-3-phosphate metabolic process [GO:0019682], ribose phosphate metabolic process [GO:0019693], GO:0030388, galactose catabolic process via UDP-galactose, Leloir pathway [GO:0033499], thiamine diphosphate metabolic process [GO:0042357], GO:0042396, phosphagen catabolic process [GO:0042397], pyridoxal phosphate metabolic process [GO:0042822], molybdopterin cofactor metabolic process [GO:0043545], inositol phosphate metabolic process [GO:0043647], deoxyribose phosphate biosynthetic process [GO:0046385], deoxyribose phosphate catabolic process [GO:0046386], glucose 6-phosphate metabolic process [GO:0051156], D-xylulose 5-phosphate metabolic process [GO:0051167], GO:0052646, chitin catabolic process to fructose 6-phosphate via glucosamine [GO:0052776], glycerol to glycerone phosphate metabolic process [GO:0061610], GO:0061720, carbamoyl phosphate metabolic process [GO:0070408], psilocybin biosynthetic process [GO:0140380], sarcinapterin metabolic process [GO:1900867], 5,6,7,8-tetrahydromethanopterin catabolic process [GO:1901284], GO:1901369, 5,6,7,8-tetrahydrosarcinapterin catabolic process [GO:1901854], D-tagatose 6-phosphate catabolic process [GO:2001059], D-glycero-D-manno-heptose 7-phosphate metabolic process [GO:2001060], methanopterin-containing compound biosynthetic process [GO:2001116], lipid X metabolic process [GO:2001289] Regulation: negatively regulated by negative regulation of phosphate metabolic process [GO:0045936]; positively regulated by positive regulation of phosphate metabolic process [GO:0045937]